{
  "gene_name": "Latent-transforming growth factor beta-binding protein 1",
  "term_id": "GO:0050436",
  "gene_symbol": "LTBP1",
  "term_label": "microfibril binding",
  "gene": "UniProtKB:Q14766"
}